nephric duct elongation [GO:0035849] (biological process) References: PMID:16216236 Sources: GOC:mtg_kidney_jan10, GOC:yaf Definition: The process in which the nephric duct grows along its axis. A nephric duct is a tube that drains a primitive kidney. Relationships: is a type of developmental growth involved in morphogenesis [GO:0060560]; is part of nephric duct morphogenesis [GO:0072178]